{
  "term_label": "potassium ion transmembrane transport",
  "term_id": "GO:0071805",
  "gene_name": "Sodium_hydrogen exchanger 4",
  "gene_symbol": "SLC9A4",
  "gene": "UniProtKB:Q6AI14"
}